cell growth mode switching, monopolar to bipolar [GO:0051523] (biological process) Relationships: is a type of GO:0061171; is a type of regulation of direction of cell growth [GO:0061389] Definition: The process in which a cell switches from monopolar cell growth to bipolar cell growth. Sources: GOC:ai Also known as: NETO, new end take off